{
  "gene": "UniProtKB:O14788",
  "gene_symbol": "TNFSF11",
  "term_id": "GO:2001238",
  "gene_name": "Tumor necrosis factor ligand superfamily member 11",
  "term_label": "positive regulation of extrinsic apoptotic signaling pathway"
}